synaptic vesicle cytoskeletal transport [GO:0099514] (biological process) Sources: GOC:dos Definition: The directed movement of synaptic vesicles along cytoskeletal fibers such as microfilaments or microtubules within a cell, powered by molecular motors. Subtypes: synaptic vesicle transport along actin filament [GO:0099506], synaptic vesicle transport along microtubule [GO:0099517] Relationships: is_a synaptic vesicle transport [GO:0048489]; is a type of vesicle cytoskeletal trafficking [GO:0099518]